{
  "gene_symbol": "PPARA",
  "gene": "UniProtKB:Q07869",
  "term_id": "GO:0000122",
  "gene_name": "Peroxisome proliferator-activated receptor alpha",
  "term_label": "negative regulation of transcription by RNA polymerase II"
}